{
  "gene_name": "RNA-binding protein 48",
  "gene": "UniProtKB:Q5RL73",
  "term_id": "UNKNOWN:0001",
  "gene_symbol": "RBM48",
  "term_label": "Unknown molecular function"
}